{
  "gene_name": "Neuronal vesicle trafficking-associated protein 1",
  "gene": "UniProtKB:P42857",
  "gene_symbol": "NSG1",
  "term_id": "GO:0016020",
  "term_label": "membrane"
}